{
  "term_id": "GO:0005886",
  "term_label": "plasma membrane",
  "gene": "UniProtKB:Q9BY67",
  "gene_symbol": "CADM1",
  "gene_name": "Cell adhesion molecule 1"
}